{
  "term_label": "Unknown molecular function",
  "term_id": "UNKNOWN:0001",
  "gene_name": "Microspherule protein 1",
  "gene_symbol": "MCRS1",
  "gene": "UniProtKB:Q96EZ8"
}